{
  "term_label": "nucleus",
  "term_id": "GO:0005634",
  "gene_symbol": "DNPH1",
  "gene": "UniProtKB:O43598",
  "gene_name": "2'-deoxynucleoside 5'-phosphate N-hydrolase 1"
}